{
  "term_label": "ribonucleoprotein complex binding",
  "gene": "UniProtKB:Q8IUD6",
  "gene_name": "E3 ubiquitin-protein ligase RNF135",
  "gene_symbol": "RNF135",
  "term_id": "GO:0043021"
}